{
  "term_label": "nuclear pore",
  "gene_name": "Nuclear envelope pore membrane protein POM 121C",
  "gene_symbol": "POM121C",
  "term_id": "GO:0005643",
  "gene": "UniProtKB:A8CG34"
}